{
  "gene": "UniProtKB:P0C264",
  "gene_name": "Uncharacterized serine_threonine-protein kinase SBK3",
  "term_id": "UNKNOWN:0003",
  "term_label": "Unknown cellular component",
  "gene_symbol": "SBK3"
}